negative regulation of response to butan-1-ol [GO:1901449] (biological process) Sources: GOC:TermGenie, GOC:mengo_curators Relationships: is_a negative regulation of response to alcohol [GO:1901420]; is a type of regulation of response to butan-1-ol [GO:1901448]; negatively regulates GO:1901422 Definition: Any process that stops, prevents or reduces the frequency, rate or extent of response to butan-1-ol. Also known as: down regulation of response to butan-1-ol, down-regulation of response to butan-1-ol, downregulation of response to butan-1-ol, inhibition of response to butan-1-ol